{
  "term_label": "Unknown cellular component",
  "gene_symbol": "UGT2B4",
  "gene": "UniProtKB:P06133",
  "gene_name": "UDP-glucuronosyltransferase 2B4",
  "term_id": "UNKNOWN:0003"
}